{
  "term_label": "Unknown cellular component",
  "gene_name": "Oxidoreductase-like domain-containing protein 1",
  "gene_symbol": "OXLD1",
  "gene": "UniProtKB:Q5BKU9",
  "term_id": "UNKNOWN:0003"
}